{
  "gene_symbol": "TCIM",
  "gene_name": "Transcriptional and immune response regulator",
  "term_label": "Notch binding",
  "gene": "UniProtKB:Q9NR00",
  "term_id": "GO:0005112"
}